maintenance of blood vessel diameter homeostasis by renin-angiotensin [GO:0002034] (biological process) Definition: The process in which the diameter of a blood vessel is changed due to activity of the renin-angiotensin system. Sources: GOC:dph, GOC:pr, GOC:tb Also known as: regulation of blood vessel size by renin-angiotensin, renin-angiotensin regulation of blood vessel size, regulation of blood vessel diameter by renin-angiotensin Relationships: is a type of renal control of peripheral vascular resistance involved in regulation of systemic arterial blood pressure [GO:0003072]; is a type of GO:0003081; is a type of blood vessel diameter maintenance [GO:0097746]